negative regulation of SMAD protein signal transduction [GO:0060392] (biological process) Definition: Any process that decreases the rate, frequency or extent of the SMAD protein signaling pathway. Relationships: is a type of regulation of SMAD protein signal transduction [GO:0060390]; is a type of GO:0090101; is a type of negative regulation of intracellular signal transduction [GO:1902532]; negatively regulates GO:0060395 Sources: GOC:BHF, GOC:dph, GOC:tb Also known as: negative regulation of SMAD protein import into nucleus, negative regulation of SMAD protein nuclear translocation